{
  "gene_name": "Methionine adenosyltransferase 2 subunit beta",
  "gene": "UniProtKB:Q9NZL9",
  "gene_symbol": "MAT2B",
  "term_id": "UNKNOWN:0001",
  "term_label": "Unknown molecular function"
}